ISG15 transferase activity [GO:0042296] (molecular function) References: PMID:12826404 Sources: GOC:mah Subtypes: GO:0061653, GO:0061662 Definition: Catalysis of the transfer of ISG15 from one protein to another via the reaction X-ISG15 + Y = Y-ISG15 + X, where both X-ISG15 and Y-ISG15 are covalent linkages. Also known as: ISG15 conjugating enzyme activity Relationships: is a type of ubiquitin-like protein transferase activity [GO:0019787]